{
  "gene": "UniProtKB:P51654",
  "gene_symbol": "GPC3",
  "gene_name": "Glypican-3",
  "term_label": "Unknown molecular function",
  "term_id": "UNKNOWN:0001"
}